{
  "gene_name": "Cytochrome P450 2B6",
  "gene_symbol": "CYP2B6",
  "gene": "UniProtKB:P20813",
  "term_label": "xenobiotic metabolic process",
  "term_id": "GO:0006805"
}